glycosphingolipid metabolic process [GO:0006687] (biological process) Sources: ISBN:0198547684 Definition: The chemical reactions and pathways involving glycosphingolipids, any compound with residues of sphingoid and at least one monosaccharide. Also known as: glycosphingolipid metabolism Subtypes: ganglioside metabolic process [GO:0001573], globoside metabolic process [GO:0001575], mannosyl-inositol phosphorylceramide metabolic process [GO:0006675], glycosylceramide metabolic process [GO:0006677], glycosphingolipid biosynthetic process [GO:0006688], glycosphingolipid catabolic process [GO:0046479] Relationships: is a type of GO:0006664; is a type of sphingolipid metabolic process [GO:0006665]